hindlimb morphogenesis [GO:0035137] (biological process) Subtypes: GO:0035116, post-embryonic hindlimb morphogenesis [GO:0035129] Sources: GOC:go_curators Definition: The process in which the anatomical structures of the hindlimb are generated and organized. Relationships: is a type of limb morphogenesis [GO:0035108]